{
  "term_id": "UNKNOWN:0002",
  "gene_symbol": "MANEAL",
  "term_label": "Unknown biological process",
  "gene_name": "Glycoprotein endo-alpha-1,2-mannosidase-like protein",
  "gene": "UniProtKB:Q5VSG8"
}